{
  "gene": "UniProtKB:Q14204",
  "gene_symbol": "DYNC1H1",
  "gene_name": "Cytoplasmic dynein 1 heavy chain 1",
  "term_id": "GO:0051959",
  "term_label": "dynein light intermediate chain binding"
}